{
  "gene": "UniProtKB:Q12906",
  "gene_symbol": "ILF3",
  "term_label": "single-stranded RNA binding",
  "term_id": "GO:0003727",
  "gene_name": "Interleukin enhancer-binding factor 3"
}